cellular response to gonadotropin stimulus [GO:0071371] (biological process) Subtypes: cellular response to human chorionic gonadotropin stimulus [GO:0044751], cellular response to follicle-stimulating hormone stimulus [GO:0071372], cellular response to luteinizing hormone stimulus [GO:0071373] Also known as: cellular response to gonadotrophin stimulus Definition: Any process that results in a change in state or activity of a cell (in terms of movement, secretion, enzyme production, gene expression, etc.) as a result of a gonadotropin stimulus. Relationships: is a type of cellular response to hormone stimulus [GO:0032870]; is a type of response to gonadotropin [GO:0034698] Sources: GOC:mah